{
  "gene_name": "Elongator complex protein 2",
  "gene": "UniProtKB:Q6IA86",
  "gene_symbol": "ELP2",
  "term_label": "Unknown biological process",
  "term_id": "UNKNOWN:0002"
}